regulation of integrin-mediated signaling pathway [GO:2001044] (biological process) Subtypes: negative regulation of integrin-mediated signaling pathway [GO:2001045], GO:2001046 Sources: GOC:obol Also known as: regulation of integrin-mediated signalling pathway Definition: Any process that modulates the frequency, rate or extent of integrin-mediated signaling pathway. Relationships: is a type of GO:0009966; RO_0002211 integrin-mediated signaling pathway [GO:0007229]